negative regulation of macrophage apoptotic process [GO:2000110] (biological process) Also known as: negative regulation of macrophage apoptosis, negative regulation of AICD, negative regulation of activation-induced cell death Sources: GOC:BHF, GOC:mtg_apoptosis Relationships: is a type of negative regulation of myeloid cell apoptotic process [GO:0033033]; is_a GO:2000107; is a type of regulation of macrophage apoptotic process [GO:2000109]; negatively regulates macrophage apoptotic process [GO:0071888] Definition: Any process that stops, prevents, or reduces the frequency, rate or extent of macrophage apoptotic process.